{
  "gene_name": "Ras-related protein Rap-1A",
  "gene": "UniProtKB:P62834",
  "term_label": "negative regulation of synaptic vesicle exocytosis",
  "term_id": "GO:2000301",
  "gene_symbol": "RAP1A"
}